{
  "gene": "UniProtKB:Q8IXF0",
  "gene_symbol": "NPAS3",
  "gene_name": "Neuronal PAS domain-containing protein 3",
  "term_label": "RNA polymerase II transcription regulatory region sequence-specific DNA binding",
  "term_id": "GO:0000977"
}